activation of meiosis [GO:0090427] (biological process) Relationships: is a type of positive regulation of meiotic nuclear division [GO:0045836] Subtypes: activation of meiosis involved in egg activation [GO:0060466] Sources: GOC:dph, GOC:tb Definition: Any process that starts the inactive process of meiosis.